{
  "term_id": "GO:0015168",
  "gene_symbol": "AQP1",
  "term_label": "glycerol transmembrane transporter activity",
  "gene_name": "Aquaporin-1",
  "gene": "UniProtKB:P29972"
}